{
  "gene": "UniProtKB:Q15323",
  "term_label": "epithelial cell differentiation",
  "gene_name": "Keratin, type I cuticular Ha1",
  "gene_symbol": "KRT31",
  "term_id": "GO:0030855"
}